{
  "term_label": "SNARE complex",
  "gene_symbol": "GOSR2",
  "gene_name": "Golgi SNAP receptor complex member 2",
  "gene": "UniProtKB:O14653",
  "term_id": "GO:0031201"
}